positive regulation of protein import into nucleus [GO:0042307] (biological process) Definition: Any process that activates or increases the frequency, rate or extent of movement of proteins from the cytoplasm into the nucleus. Also known as: positive regulation of protein import into cell nucleus, positive regulation of protein transport from cytoplasm to nucleus, positive regulation of protein-nucleus import, up regulation of protein import into nucleus, up-regulation of protein import into nucleus, upregulation of protein import into nucleus, activation of protein import into nucleus, stimulation of protein import into nucleus Sources: GOC:jl Relationships: is a type of regulation of protein import into nucleus [GO:0042306]; is a type of positive regulation of nucleocytoplasmic transport [GO:0046824]; is a type of positive regulation of intracellular protein transport [GO:0090316]; is a type of positive regulation of protein localization to nucleus [GO:1900182]; positively regulates protein import into nucleus [GO:0006606]